sirohydrochlorin cobaltochelatase activity [GO:0016852] (molecular function) Definition: Catalysis of the reaction: sirohydrochlorin + Co2+ = cobalt-sirohydrochlorin + 2 H+. Also known as: anaerobic cobalt chelatase activity, cobaltochelatase, cobalt-sirohydrochlorin cobalt-lyase (sirohydrochlorin-forming), sirohydrochlorin cobalt-lyase activity Sources: RHEA:15893 Relationships: is a type of lyase activity [GO:0016829]